{
  "gene": "UniProtKB:Q9BXF3",
  "term_id": "GO:0007338",
  "gene_name": "Chromatin remodeling regulator CECR2",
  "term_label": "single fertilization",
  "gene_symbol": "CECR2"
}